tetrapeptide import across plasma membrane [GO:1901583] (BP) Definition: The directed movement of a tetrapeptide from outside of a cell, across the plasma membrane and into the cytosol. References: PMID:22226946 Sources: GOC:TermGenie Relationships: is a type of GO:0140205 Also known as: tetrapeptide transmembrane transport, tetrapeptide membrane transport Note: Note that this term is not intended for use in annotating lateral movement within membranes.